sequoyitol dehydrogenase activity [GO:0050280] (molecular function) Relationships: is a type of oxidoreductase activity, acting on the CH-OH group of donors, NAD or NADP as acceptor [GO:0016616] Also known as: 5-O-methyl-myo-inositol:NAD+ oxidoreductase activity Sources: EC:1.1.1.143, RHEA:11300 Definition: Catalysis of the reaction: 1D-5-O-methyl-myo-inositol + NAD+ = 2D-5-O-methyl-2,3,5/4,6-pentahydroxycyclohexanone + H+ + NADH.